{
  "gene_name": "Testis-expressed protein 11",
  "gene_symbol": "TEX11",
  "gene": "UniProtKB:Q8IYF3",
  "term_label": "reciprocal meiotic recombination",
  "term_id": "GO:0007131"
}